{
  "term_id": "GO:0005634",
  "gene_symbol": "FGF1",
  "term_label": "nucleus",
  "gene_name": "Fibroblast growth factor 1",
  "gene": "UniProtKB:P05230"
}